regulation of plasma lipoprotein oxidation [GO:0034444] (biological process) Definition: Any process that modulates the frequency, rate or extent of lipoprotein oxidation, occurring in the blood plasma. Subtypes: negative regulation of plasma lipoprotein oxidation [GO:0034445] Also known as: regulation of plasma lipoprotein particle oxidation Sources: GOC:BHF, GOC:mah Relationships: is a type of GO:0051128; is a type of GO:0051239; regulates plasma lipoprotein particle oxidation [GO:0034441]